{
  "gene_name": "Solute carrier family 22 member 2",
  "term_label": "Unknown molecular function",
  "gene": "UniProtKB:O15244",
  "term_id": "UNKNOWN:0001",
  "gene_symbol": "SLC22A2"
}